L-cystine transmembrane transport from lysosomal lumen to cytosol [GO:1904919] (biological process) Also known as: transmembrane L-cystine transport from lysosomal lumen to cytosol Relationships: is a type of L-cystine transport [GO:0015811]; is a type of neutral amino acid transmembrane export from vacuole [GO:0034489]; is a type of transmembrane transport from lysosomal lumen to cytosol [GO:0170063]; is a type of L-alpha-amino acid transmembrane transport [GO:1902475] References: PMID:22822152 Sources: GOC:TermGenie, GOC:kmv, GO_REF:0000078 Definition: The directed movement of L-cystine from the lysosomal lumen across the lysosomal membrane and into the cytosol.